diacylglycerol diphosphate phosphatase activity [GO:0000810] (molecular function) Also known as: DGPP phosphatase activity, DGPP phosphohydrolase activity, diacylglycerol pyrophosphate phosphatase activity Definition: Catalysis of the reaction: a 1,2-diacyl-sn-glycerol 3-diphosphate + H2O = a 1,2-diacyl-sn-glycerol 3-phosphate + phosphate. References: PMID:8567632, PMID:9452443 Sources: GOC:kad, RHEA:27449 Relationships: is a type of pyrophosphatase activity [GO:0016462]